post-embryonic digestive tract morphogenesis [GO:0048621] (biological process) Relationships: is a type of post-embryonic animal morphogenesis [GO:0009886]; is part of digestive tract morphogenesis [GO:0048546] Sources: GOC:jid, GOC:rc Also known as: post-embryonic gut morphogenesis Definition: The process, occurring during the post-embryonic phase, by which the anatomical structures of the digestive tract are generated and organized. The digestive tract is the anatomical structure through which food passes and is processed.